{
  "gene": "UniProtKB:Q96PL5",
  "gene_name": "Erythroid membrane-associated protein",
  "term_label": "T cell receptor signaling pathway",
  "gene_symbol": "ERMAP",
  "term_id": "GO:0050852"
}